Atg12 transferase activity [GO:0019777] (molecular function) References: PMID:12826404 Sources: GOC:mah Definition: Catalysis of the transfer of ATG12 from one protein to another via the reaction X-ATG12 + Y = Y-ATG12 + X, where both X-ATG12 and Y-ATG12 are covalent linkages. Relationships: is_a GO:0019787 Subtypes: GO:0061651, GO:0061660 Also known as: APG12 conjugating enzyme activity, APG12 ligase activity, Atg12 conjugating enzyme activity, Atg12 ligase activity